{
  "gene_name": "Tumor necrosis factor receptor superfamily member 14",
  "term_id": "GO:2000406",
  "term_label": "positive regulation of T cell migration",
  "gene_symbol": "TNFRSF14",
  "gene": "UniProtKB:Q92956"
}